{
  "gene_symbol": "MENT",
  "term_label": "regulation of cell population proliferation",
  "gene": "UniProtKB:Q9BUN1",
  "term_id": "GO:0042127",
  "gene_name": "Protein MENT"
}